regulation of protein binding [GO:0043393] (biological process) Subtypes: negative regulation of protein binding [GO:0032091], positive regulation of protein binding [GO:0032092], GO:1900120 Relationships: is a type of GO:0051098; regulates protein binding [GO:0005515] Definition: Any process that modulates the frequency, rate or extent of protein binding. Sources: GOC:go_curators